{
  "term_label": "histone binding",
  "gene": "UniProtKB:Q92688",
  "gene_name": "Acidic leucine-rich nuclear phosphoprotein 32 family member B",
  "term_id": "GO:0042393",
  "gene_symbol": "ANP32B"
}